{
  "gene": "UniProtKB:Q9NRC9",
  "gene_symbol": "OTOR",
  "term_label": "Unknown molecular function",
  "term_id": "UNKNOWN:0001",
  "gene_name": "Otoraplin"
}